{
  "gene_symbol": "PIR",
  "term_label": "monocyte differentiation",
  "gene_name": "Pirin",
  "gene": "UniProtKB:O00625",
  "term_id": "GO:0030224"
}